{
  "gene": "UniProtKB:O15539",
  "term_label": "cytoplasmic side of plasma membrane",
  "gene_symbol": "RGS5",
  "term_id": "GO:0009898",
  "gene_name": "Regulator of G-protein signaling 5"
}